{
  "gene_name": "Plasminogen-like protein B",
  "term_id": "UNKNOWN:0001",
  "gene": "UniProtKB:Q02325",
  "gene_symbol": "PLGLB2",
  "term_label": "Unknown molecular function"
}